{
  "gene_name": "Probable G-protein coupled receptor 146",
  "term_label": "Unknown molecular function",
  "gene_symbol": "GPR146",
  "gene": "UniProtKB:Q96CH1",
  "term_id": "UNKNOWN:0001"
}